{
  "term_id": "GO:0005085",
  "gene_symbol": "MON2",
  "gene_name": "Protein MON2 homolog",
  "term_label": "guanyl-nucleotide exchange factor activity",
  "gene": "UniProtKB:Q7Z3U7"
}